{
  "term_label": "Unknown biological process",
  "term_id": "UNKNOWN:0002",
  "gene_name": "Uncharacterized protein encoded by LINC03043",
  "gene_symbol": "LINC03043",
  "gene": "UniProtKB:A4D0Y5"
}